negative regulation of male germ cell proliferation [GO:2000255] (biological process) Relationships: is a type of negative regulation of germ cell proliferation [GO:1905937]; is a type of negative regulation of reproductive process [GO:2000242]; is a type of GO:2000254; negatively regulates male germ cell proliferation [GO:0002176] Definition: Any process that stops, prevents or reduces the frequency, rate or extent of male germ cell proliferation. Sources: GOC:obol